{
  "term_label": "peptide YY receptor activity",
  "gene_name": "Neuropeptide Y receptor type 4-2",
  "gene_symbol": "NPY4R2",
  "gene": "UniProtKB:P0DQD5",
  "term_id": "GO:0001601"
}